{
  "gene_symbol": "CTNND1",
  "term_label": "plasma membrane",
  "term_id": "GO:0005886",
  "gene_name": "Catenin delta-1",
  "gene": "UniProtKB:O60716"
}